{
  "gene": "UniProtKB:Q9Y6C5",
  "gene_name": "Protein patched homolog 2",
  "term_id": "GO:0005119",
  "term_label": "smoothened binding",
  "gene_symbol": "PTCH2"
}